{
  "gene": "UniProtKB:Q92521",
  "gene_name": "GPI mannosyltransferase 3",
  "gene_symbol": "PIGB",
  "term_label": "alpha-1,2-mannosyltransferase activity",
  "term_id": "GO:0000026"
}